D-glucose import across plasma membrane [GO:0098708] (biological process) Sources: GOC:dos Also known as: glucose import across plasma membrane, glucose import into cell, high affinity glucose import Relationships: is a type of GO:0140271; is a type of D-glucose transmembrane transport [GO:1904659] Definition: The directed movement of D-glucose from outside of a cell, across the plasma membrane and into the cytosol.